{
  "gene_name": "Homeobox protein TGIF2",
  "gene": "UniProtKB:Q9GZN2",
  "term_label": "DNA-binding transcription repressor activity, RNA polymerase II-specific",
  "gene_symbol": "TGIF2",
  "term_id": "GO:0001227"
}